{
  "gene_symbol": "TH",
  "term_id": "GO:0042421",
  "gene": "UniProtKB:P07101",
  "gene_name": "Tyrosine 3-monooxygenase",
  "term_label": "norepinephrine biosynthetic process"
}